{
  "term_id": "GO:0016460",
  "gene_name": "Myosin light chain 1_3, skeletal muscle isoform",
  "gene_symbol": "MYL1",
  "term_label": "myosin II complex",
  "gene": "UniProtKB:P05976"
}